{
  "gene_symbol": "TMEM167A",
  "term_label": "Unknown molecular function",
  "term_id": "UNKNOWN:0001",
  "gene": "UniProtKB:Q8TBQ9",
  "gene_name": "Protein kish-A"
}